{
  "term_label": "Unknown cellular component",
  "gene": "UniProtKB:Q6ZQT7",
  "term_id": "UNKNOWN:0003",
  "gene_name": "Putative uncharacterized protein FLJ44672",
  "gene_symbol": "Q6ZQT7"
}